{
  "gene_name": "Neuromedin-U",
  "term_id": "GO:0050806",
  "gene_symbol": "NMU",
  "term_label": "positive regulation of synaptic transmission",
  "gene": "UniProtKB:P48645"
}